{
  "term_id": "UNKNOWN:0002",
  "gene_name": "Aminoacyl tRNA synthase complex-interacting multifunctional protein 1",
  "gene": "UniProtKB:Q12904",
  "gene_symbol": "AIMP1",
  "term_label": "Unknown biological process"
}